magnetosome assembly [GO:0140923] (biological process) Also known as: magnetosome formation Definition: The aggregation, arrangement and bonding together of a set of components to form a magnetosome. Magnetosomes are specialized organelles for magnetic navigation that comprise membrane-enveloped, nano-sized crystals of a magnetic iron mineral; they are formed by a diverse group of magnetotactic bacteria (MTB). Relationships: is a type of GO:0070925 References: PMID:19575557, PMID:34723168